{
  "gene_symbol": "PPP3CB",
  "term_label": "calmodulin-dependent protein phosphatase activity",
  "gene_name": "Serine_threonine-protein phosphatase 2B catalytic subunit beta isoform",
  "term_id": "GO:0033192",
  "gene": "UniProtKB:P16298"
}